{
  "gene_symbol": "GJE1",
  "gene_name": "Putative gap junction epsilon-1 protein",
  "term_label": "connexin complex",
  "term_id": "GO:0005922",
  "gene": "UniProtKB:A6NN92"
}